{
  "term_id": "GO:0016064",
  "term_label": "immunoglobulin mediated immune response",
  "gene_symbol": "IGHV1-69-2",
  "gene_name": "Immunoglobulin heavy variable 1-69-2",
  "gene": "UniProtKB:A0A0G2JMI3"
}